{
  "term_label": "nucleus",
  "term_id": "GO:0005634",
  "gene_name": "Zinc finger protein 729",
  "gene": "UniProtKB:A6NN14",
  "gene_symbol": "ZNF729"
}